{
  "gene_symbol": "CAMK1G",
  "term_id": "GO:0005516",
  "gene": "UniProtKB:Q96NX5",
  "term_label": "calmodulin binding",
  "gene_name": "Calcium_calmodulin-dependent protein kinase type 1G"
}